{
  "term_label": "embryonic organ development",
  "gene_symbol": "TEAD2",
  "gene_name": "Transcriptional enhancer factor TEF-4",
  "gene": "UniProtKB:Q15562",
  "term_id": "GO:0048568"
}